{
  "gene": "UniProtKB:Q92556",
  "term_label": "plasma membrane",
  "term_id": "GO:0005886",
  "gene_name": "Engulfment and cell motility protein 1",
  "gene_symbol": "ELMO1"
}